{
  "term_id": "GO:0099572",
  "gene": "UniProtKB:Q9Y2H0",
  "gene_name": "Disks large-associated protein 4",
  "gene_symbol": "DLGAP4",
  "term_label": "postsynaptic specialization"
}